{
  "term_id": "GO:0031982",
  "term_label": "vesicle",
  "gene_symbol": "SLC34A3",
  "gene_name": "Sodium-dependent phosphate transport protein 2C",
  "gene": "UniProtKB:Q8N130"
}